{
  "term_id": "UNKNOWN:0001",
  "gene_symbol": "AIG1",
  "gene_name": "Androgen-induced gene 1 protein",
  "term_label": "Unknown molecular function",
  "gene": "UniProtKB:Q9NVV5"
}